{
  "term_label": "translation initiation factor activity",
  "gene": "UniProtKB:P60842",
  "gene_name": "Eukaryotic initiation factor 4A-I",
  "term_id": "GO:0003743",
  "gene_symbol": "EIF4A1"
}